{
  "gene_name": "Lysine-specific demethylase PHF2",
  "term_id": "GO:0006357",
  "gene": "UniProtKB:O75151",
  "term_label": "regulation of transcription by RNA polymerase II",
  "gene_symbol": "PHF2"
}